natural killer cell tolerance induction [GO:0002519] (biological process) Also known as: NK cell tolerance induction Regulation: regulated by regulation of natural killer cell tolerance induction [GO:0002871]; negatively regulated by negative regulation of natural killer cell tolerance induction [GO:0002872]; positively regulated by positive regulation of natural killer cell tolerance induction [GO:0002873] References: PMID:16546094 Sources: GOC:jal Relationships: is a type of tolerance induction [GO:0002507] Definition: Tolerance induction of natural killer cells.